deoxyribonucleotide biosynthetic process [GO:0009263] (biological process) Definition: The chemical reactions and pathways resulting in the formation of a deoxyribonucleotide, a compound consisting of deoxyribonucleoside (a base linked to a deoxyribose sugar) esterified with a phosphate group at either the 3' or 5'-hydroxyl group of the sugar. Sources: GOC:go_curators, ISBN:0198506732 Also known as: deoxyribonucleotide anabolism, deoxyribonucleotide biosynthesis, deoxyribonucleotide formation, deoxyribonucleotide synthesis Relationships: is a type of nucleotide biosynthetic process [GO:0009165]; is a type of deoxyribonucleotide metabolic process [GO:0009262]; is a type of carbohydrate derivative biosynthetic process [GO:1901137] Subtypes: 2'-deoxyribonucleotide biosynthetic process [GO:0009265]